protein localization to microtubule cytoskeleton [GO:0072698] (biological process) Definition: A cellular protein localization process in which a protein is transported to, or maintained at, a location within the microtubule cytoskeleton. Also known as: protein localisation to microtubule cytoskeleton Relationships: is a type of GO:0044380 Subtypes: protein localization to microtubule [GO:0035372], GO:0072699, protein localization to mitotic spindle [GO:1902480], protein localization to meiotic spindle [GO:1905359], protein localization to microtubule organizing center [GO:1905508] Sources: GOC:mah